{
  "term_label": "Unknown biological process",
  "term_id": "UNKNOWN:0002",
  "gene_name": "Thymosin beta-15C",
  "gene": "UniProtKB:P0DX04",
  "gene_symbol": "TMSB15C"
}